{
  "gene_name": "Lysine-specific demethylase 4C",
  "term_label": "regulation of gene expression",
  "gene": "UniProtKB:Q9H3R0",
  "term_id": "GO:0010468",
  "gene_symbol": "KDM4C"
}